D-glucarate transmembrane transport [GO:0042870] (biological process) Relationships: is_a carbohydrate transmembrane transport [GO:0034219]; is_a aldarate transmembrane transport [GO:0042869] Also known as: D-glucarate transport Definition: The process in which D-glucarate, the D-enantiomer of glucarate, is transported across a lipid bilayer, from one side of a membrane to the other. Sources: GOC:jl, GOC:jsg, GOC:mah, ISBN:0198506732